{
  "term_id": "GO:0004029",
  "gene_name": "Mitochondrial 10-formyltetrahydrofolate dehydrogenase",
  "gene_symbol": "ALDH1L2",
  "term_label": "aldehyde dehydrogenase (NAD+) activity",
  "gene": "UniProtKB:Q3SY69"
}